{
  "gene_name": "Myeloid zinc finger 1",
  "term_label": "regulation of DNA-templated transcription",
  "gene": "UniProtKB:P28698",
  "term_id": "GO:0006355",
  "gene_symbol": "MZF1"
}